{
  "term_id": "UNKNOWN:0001",
  "gene_name": "Putative uncharacterized protein UNQ6494_PRO21346",
  "gene": "UniProtKB:Q6UXR6",
  "gene_symbol": "UNQ6494_PRO21346",
  "term_label": "Unknown molecular function"
}